{
  "term_id": "UNKNOWN:0002",
  "gene": "UniProtKB:A4QN01",
  "gene_name": "Putative uncharacterized protein encoded by LINC01553",
  "term_label": "Unknown biological process",
  "gene_symbol": "LINC01553"
}